{
  "gene_name": "Serine_threonine-protein kinase BRSK1",
  "term_label": "centrosome",
  "term_id": "GO:0005813",
  "gene_symbol": "BRSK1",
  "gene": "UniProtKB:Q8TDC3"
}